uroporphyrinogen-III synthase activity [GO:0004852] (molecular function) Definition: Catalysis of the reaction: hydroxymethylbilane = H2O + uroporphyrinogen III. Sources: EC:4.2.1.75, RHEA:18965 Also known as: URO-synthase activity, hydroxymethylbilane hydro-lyase (cyclizing) activity, hydroxymethylbilane hydro-lyase (cyclizing; uroporphyrinogen-III-forming), porphobilinogenase activity, uroporphyrinogen III cosynthase activity, uroporphyrinogen isomerase activity, uroporphyrinogen-III cosynthase activity, uroporphyrinogen-III cosynthetase activity Relationships: is a type of hydro-lyase activity [GO:0016836]